{
  "gene": "UniProtKB:Q6A163",
  "gene_name": "Keratin, type I cytoskeletal 39",
  "term_label": "cytoskeleton",
  "term_id": "GO:0005856",
  "gene_symbol": "KRT39"
}